{
  "gene_name": "Thrombopoietin receptor",
  "gene": "UniProtKB:P40238",
  "gene_symbol": "MPL",
  "term_id": "GO:0009897",
  "term_label": "external side of plasma membrane"
}